AP-type membrane coat adaptor complex [GO:0030119] (cellular component) Definition: Any of several heterotetrameric complexes that link clathrin (or another coat-forming molecule, as hypothesized for AP-3 and AP-4) to a membrane surface; they are found on coated pits and coated vesicles, and mediate sorting of cargo proteins into vesicles. Each AP complex contains two large (a beta and one of either an alpha, gamma, delta, or epsilon) subunits (110-130 kDa), a medium (mu) subunit (approximately 50 kDa), and a small (sigma) subunit (15-20 kDa). Also known as: clathrin adaptor References: PMID:10611976, PMID:15473838 Sources: GOC:mah Relationships: is a type of membrane protein complex [GO:0098796]; is part of membrane coat [GO:0030117] Subtypes: AP-3 adaptor complex [GO:0030123], GO:0030124, clathrin adaptor complex [GO:0030131], AP-5 adaptor complex [GO:0044599]